double-strand break repair via single-strand annealing [GO:0045002] (biological process) Definition: Repair of a DSB made between two repeated sequences oriented in the same direction occurs primarily by the single strand annealing pathway. The ends of the break are processed by a 5' to 3' exonuclease, exposing complementary single-strand regions of the direct repeats that can anneal, resulting in a deletion of the unique DNA between the direct repeats. References: PMID:11606529 Relationships: is a type of double-strand break repair [GO:0006302] Regulation: negatively regulated by negative regulation of double-strand break repair via single-strand annealing [GO:1901291]